poly(A)+ mRNA export from nucleus [GO:0016973] (biological process) Relationships: is a type of mRNA export from nucleus [GO:0006406] Definition: The directed movement of poly(A)+ mRNA out of the nucleus into the cytoplasm. Also known as: poly(A) mRNA export from nucleus, poly(A)+ mRNA export from cell nucleus, poly(A)+ mRNA export out of nucleus, poly(A)+ mRNA transport from nucleus to cytoplasm, poly(A)+ mRNA-nucleus export, polyadenylated mRNA export from nucleus Sources: GOC:ai